{
  "gene": "UniProtKB:P15056",
  "gene_name": "Serine_threonine-protein kinase B-raf",
  "term_id": "GO:0005739",
  "gene_symbol": "BRAF",
  "term_label": "mitochondrion"
}